{
  "gene": "UniProtKB:O75264",
  "term_label": "Unknown biological process",
  "term_id": "UNKNOWN:0002",
  "gene_name": "Small integral membrane protein 24",
  "gene_symbol": "SMIM24"
}